positive regulation of transformation of host cell by virus [GO:1904189] (biological process) Also known as: positive regulation of viral transformation, positive regulation of viral transformation of host cell, up regulation of transformation of host cell by virus, up regulation of viral transformation, up regulation of viral transformation of host cell, up-regulation of transformation of host cell by virus, up-regulation of viral transformation, up-regulation of viral transformation of host cell, upregulation of transformation of host cell by virus, upregulation of viral transformation, upregulation of viral transformation of host cell, activation of transformation of host cell by virus, activation of viral transformation, activation of viral transformation of host cell Relationships: is a type of positive regulation of biological process [GO:0048518]; is a type of regulation of transformation of host cell by virus [GO:1904187]; positively regulates GO:0019087 Definition: Any process that activates or increases the frequency, rate or extent of transformation of host cell by virus. References: PMID:12200142 Sources: GOC:TermGenie, GO_REF:0000058